{
  "gene_symbol": "AASDH",
  "term_label": "Unknown molecular function",
  "term_id": "UNKNOWN:0001",
  "gene_name": "Beta-alanine-activating enzyme",
  "gene": "UniProtKB:Q4L235"
}